carnosine metabolic process [GO:0035498] (biological process) Subtypes: carnosine biosynthetic process [GO:0035499] Also known as: carnosine metabolism Definition: The chemical reactions and pathways involving the dipeptide beta-alanyl-L-histidine (carnosine). References: PMID:20097752 Relationships: is a type of GO:0006520; is a type of carboxylic acid metabolic process [GO:0019752]; is a type of amide metabolic process [GO:0043603]